{
  "gene_symbol": "ZNF528",
  "gene_name": "Zinc finger protein 528",
  "gene": "UniProtKB:Q3MIS6",
  "term_label": "regulation of transcription by RNA polymerase II",
  "term_id": "GO:0006357"
}